{
  "gene_symbol": "ACTG1",
  "term_id": "GO:0019901",
  "gene": "UniProtKB:P63261",
  "term_label": "protein kinase binding",
  "gene_name": "Actin, cytoplasmic 2"
}